{
  "term_id": "GO:0004930",
  "gene": "UniProtKB:Q8TCW9",
  "gene_symbol": "PROKR1",
  "gene_name": "Prokineticin receptor 1",
  "term_label": "G protein-coupled receptor activity"
}